filamentous growth of a multicellular organism [GO:0044181] (biological process) Sources: GOC:mtg_cambridge_2009 Relationships: is a type of filamentous growth [GO:0030447]; is_a developmental growth involved in morphogenesis [GO:0060560] Definition: The process in which a multicellular organism grows in a threadlike, filamentous shape.